{
  "gene_name": "Homeobox protein SEBOX",
  "gene_symbol": "SEBOX",
  "term_label": "Unknown cellular component",
  "term_id": "UNKNOWN:0003",
  "gene": "UniProtKB:Q9HB31"
}